negative regulation of leukocyte adhesion to arterial endothelial cell [GO:1904998] (biological process) Definition: Any process that stops, prevents or reduces the frequency, rate or extent of leukocyte adhesion to arterial endothelial cell. References: PMID:22267480 Sources: GOC:BHF, GOC:BHF_miRNA, GOC:TermGenie, GOC:bc, GO_REF:0000058 Also known as: down regulation of leukocyte adhesion to arterial endothelial cell, down-regulation of leukocyte adhesion to arterial endothelial cell, downregulation of leukocyte adhesion to arterial endothelial cell, inhibition of leukocyte adhesion to arterial endothelial cell Relationships: is a type of GO:1904995; is a type of regulation of leukocyte adhesion to arterial endothelial cell [GO:1904997]; RO_0002212 leukocyte adhesion to arterial endothelial cell [GO:0061757]